{
  "term_label": "Unknown biological process",
  "gene": "UniProtKB:Q96EK6",
  "term_id": "UNKNOWN:0002",
  "gene_symbol": "GNPNAT1",
  "gene_name": "Glucosamine 6-phosphate N-acetyltransferase"
}